{
  "term_label": "plasma membrane",
  "gene": "UniProtKB:Q08881",
  "term_id": "GO:0005886",
  "gene_name": "Tyrosine-protein kinase ITK_TSK",
  "gene_symbol": "ITK"
}